{
  "term_id": "GO:0006325",
  "gene": "UniProtKB:P23527",
  "gene_symbol": "H2BC17",
  "gene_name": "Histone H2B type 1-O",
  "term_label": "chromatin organization"
}